{
  "gene_name": "Programmed cell death 1 ligand 2",
  "term_id": "UNKNOWN:0001",
  "term_label": "Unknown molecular function",
  "gene": "UniProtKB:Q9BQ51",
  "gene_symbol": "PDCD1LG2"
}